{
  "gene": "UniProtKB:Q9NVE4",
  "gene_name": "Coiled-coil domain-containing protein 87",
  "term_label": "Unknown molecular function",
  "gene_symbol": "CCDC87",
  "term_id": "UNKNOWN:0001"
}